{
  "term_label": "cell-matrix adhesion",
  "gene_symbol": "FERMT1",
  "term_id": "GO:0007160",
  "gene": "UniProtKB:Q9BQL6",
  "gene_name": "Fermitin family homolog 1"
}